{
  "gene_name": "T-box transcription factor TBX4",
  "term_id": "GO:0000785",
  "gene": "UniProtKB:P57082",
  "gene_symbol": "TBX4",
  "term_label": "chromatin"
}